{
  "term_label": "peptide antigen binding",
  "gene_name": "HLA class II histocompatibility antigen, DM alpha chain",
  "gene": "UniProtKB:P28067",
  "gene_symbol": "HLA-DMA",
  "term_id": "GO:0042605"
}